{
  "term_id": "UNKNOWN:0002",
  "gene_symbol": "SETD1B",
  "gene": "UniProtKB:Q9UPS6",
  "term_label": "Unknown biological process",
  "gene_name": "Histone-lysine N-methyltransferase SETD1B"
}